integrin alpha2-beta1 complex [GO:0034666] (cellular component) Definition: An integrin complex that comprises one alpha2 subunit and one beta1 subunit. References: PMID:12297042 Also known as: VLA-2 complex, ITGA2-ITGB1 complex Relationships: is a type of integrin complex [GO:0008305]